disaccharide transmembrane transporter activity [GO:0015154] (molecular function) Definition: Enables the transfer of disaccharide from one side of a membrane to the other. Relationships: is a type of oligosaccharide transmembrane transporter activity [GO:0015157]; is part of disaccharide transport [GO:0015766] Subtypes: GO:0005363, GO:0008515, GO:0015155, GO:0015156, trehalose transmembrane transporter activity [GO:0015574], GO:0019191 Sources: GOC:jl, GOC:mtg_transport, ISBN:0815340729